{
  "term_id": "GO:0005245",
  "gene_symbol": "CACNA2D4",
  "gene_name": "Voltage-dependent calcium channel subunit alpha-2_delta-4",
  "term_label": "voltage-gated calcium channel activity",
  "gene": "UniProtKB:Q7Z3S7"
}